late endosome to vacuole transport [GO:0045324] (biological process) Definition: The directed movement of substances from late endosomes to the vacuole. In yeast, after transport to the prevacuolar compartment, endocytic content is delivered to the late endosome and on to the vacuole. This pathway is analogous to endosome to lysosome transport. References: PMID:11872141 Relationships: is a type of vacuolar transport [GO:0007034]; is a type of GO:0016192 Subtypes: late endosome to vacuole transport via multivesicular body sorting pathway [GO:0032511], late endosome to lysosome transport via multivesicular body sorting pathway [GO:0061764]